{
  "gene_name": "Neural cell adhesion molecule L1-like protein",
  "term_id": "UNKNOWN:0002",
  "term_label": "Unknown biological process",
  "gene": "UniProtKB:O00533",
  "gene_symbol": "CHL1"
}